mitral valve morphogenesis [GO:0003183] (biological process) Definition: The process in which the structure of the mitral valve is generated and organized. Relationships: is a type of GO:0003181; is part of GO:0003174 Sources: GOC:mtg_heart